positive regulation of heart rate by circulating epinephrine [GO:0003111] (BP) Definition: The process in which the secretion of epinephrine into the bloodstream increases the rate of heart muscle contraction. Also known as: positive regulation of heart rate by circulating adrenaline Relationships: is a type of positive regulation of heart rate by epinephrine [GO:0003065] Sources: GOC:mtg_cardio